{
  "gene_name": "Hemojuvelin",
  "term_id": "GO:0030509",
  "term_label": "BMP signaling pathway",
  "gene": "UniProtKB:Q6ZVN8",
  "gene_symbol": "HJV"
}